single cytosine insertion binding [GO:0032141] (molecular function) Relationships: is a type of single base insertion or deletion binding [GO:0032138] Definition: Binding to a double-stranded DNA region containing a single cytosine insertion or a deletion that results in an unpaired cytosine. Sources: GOC:mah, GOC:vk